{
  "gene_name": "Interleukin enhancer-binding factor 3",
  "term_id": "UNKNOWN:0002",
  "gene_symbol": "ILF3",
  "gene": "UniProtKB:Q12906",
  "term_label": "Unknown biological process"
}